{
  "gene_name": "Nesprin-3",
  "term_label": "cytoplasm",
  "term_id": "GO:0005737",
  "gene": "UniProtKB:Q6ZMZ3",
  "gene_symbol": "SYNE3"
}